{
  "gene_name": "Claspin",
  "gene_symbol": "CLSPN",
  "gene": "UniProtKB:Q9HAW4",
  "term_id": "GO:0010997",
  "term_label": "anaphase-promoting complex binding"
}